{
  "term_label": "plasma membrane",
  "gene_name": "Alpha-2-macroglobulin receptor-associated protein",
  "term_id": "GO:0005886",
  "gene": "UniProtKB:P30533",
  "gene_symbol": "LRPAP1"
}